negative regulation of hemoglobin biosynthetic process [GO:0046986] (biological process) Sources: GOC:ai Definition: Any process that stops, prevents, or reduces the frequency, rate or extent of the chemical reactions and pathways resulting in the formation of hemoglobin, an oxygen carrying, conjugated protein containing four heme groups and globin. Also known as: down regulation of hemoglobin biosynthetic process, down-regulation of hemoglobin biosynthetic process, downregulation of hemoglobin biosynthetic process, negative regulation of haemoglobin biosynthesis, negative regulation of haemoglobin biosynthetic process, negative regulation of hemoglobin anabolism, negative regulation of hemoglobin biosynthesis, negative regulation of hemoglobin formation, negative regulation of hemoglobin synthesis, inhibition of hemoglobin biosynthetic process Relationships: is a type of GO:0010558; is a type of regulation of hemoglobin biosynthetic process [GO:0046984]; is a type of negative regulation of protein metabolic process [GO:0051248]; negatively regulates GO:0042541